{
  "gene_name": "Uncharacterized protein ADAMTSL4-AS1",
  "term_id": "UNKNOWN:0001",
  "gene_symbol": "ADAMTSL4-AS1",
  "term_label": "Unknown molecular function",
  "gene": "UniProtKB:Q5T5F5"
}